{
  "gene": "UniProtKB:Q9ULJ3",
  "term_id": "GO:0005634",
  "gene_symbol": "ZBTB21",
  "term_label": "nucleus",
  "gene_name": "Zinc finger and BTB domain-containing protein 21"
}